{
  "gene_name": "Dapper homolog 2",
  "term_id": "GO:1900108",
  "gene": "UniProtKB:Q5SW24",
  "term_label": "negative regulation of nodal signaling pathway",
  "gene_symbol": "DACT2"
}